{
  "gene": "UniProtKB:Q15466",
  "term_label": "negative regulation of transcription by RNA polymerase II",
  "gene_name": "Nuclear receptor subfamily 0 group B member 2",
  "term_id": "GO:0000122",
  "gene_symbol": "NR0B2"
}